{
  "term_id": "GO:2000766",
  "gene_symbol": "CPEB4",
  "gene_name": "Cytoplasmic polyadenylation element-binding protein 4",
  "gene": "UniProtKB:Q17RY0",
  "term_label": "negative regulation of cytoplasmic translation"
}